{
  "term_id": "GO:0031146",
  "gene_symbol": "FBXL6",
  "gene_name": "F-box_LRR-repeat protein 6",
  "term_label": "SCF-dependent proteasomal ubiquitin-dependent protein catabolic process",
  "gene": "UniProtKB:Q8N531"
}